response to fructose [GO:0009750] (biological process) Also known as: response to fructose stimulus Sources: GOC:jl Subtypes: cellular response to fructose stimulus [GO:0071332] Relationships: is a type of response to hexose [GO:0009746] Definition: Any process that results in a change in state or activity of a cell or an organism (in terms of movement, secretion, enzyme production, gene expression, etc.) as a result of a fructose stimulus.